{
  "gene_symbol": "SPRY2",
  "term_id": "GO:0004860",
  "gene": "UniProtKB:O43597",
  "gene_name": "Protein sprouty homolog 2",
  "term_label": "protein kinase inhibitor activity"
}